{
  "gene_name": "Sodium-dependent noradrenaline transporter",
  "term_label": "amino acid transport",
  "gene_symbol": "SLC6A2",
  "term_id": "GO:0006865",
  "gene": "UniProtKB:P23975"
}